{
  "term_label": "signal transduction",
  "gene_symbol": "CD300A",
  "gene": "UniProtKB:Q9UGN4",
  "gene_name": "CMRF35-like molecule 8",
  "term_id": "GO:0007165"
}